{
  "gene": "UniProtKB:P35968",
  "gene_symbol": "KDR",
  "term_label": "regulation of MAPK cascade",
  "term_id": "GO:0043408",
  "gene_name": "Vascular endothelial growth factor receptor 2"
}